violaxanthin oxygenase activity [GO:0102785] (molecular function) Relationships: is a type of oxidoreductase activity, acting on single donors with incorporation of molecular oxygen, incorporation of two atoms of oxygen [GO:0016702] Definition: Catalysis of the reaction: violaxanthin + 2 O2 = 2 5,6-epoxy-3-hydroxy-9-apo-beta-caroten-9-one + 4,9-dimethyldodeca-2,4,6,8,10-pentaenedial. References: PMID:11316814 Sources: GOC:pz